actomyosin structure organization [GO:0031032] (biological process) Definition: A process that is carried out at the cellular level which results in the assembly, arrangement of constituent parts, or disassembly of cytoskeletal structures containing both actin and myosin or paramyosin. The myosin may be organized into filaments. Sources: GOC:dph, GOC:jl, GOC:mah Also known as: actomyosin organization, actomyosin structure organisation, actomyosin structure organization and biogenesis Note: Note that this term is a child of 'actin cytoskeleton organization and biogenesis ; GO:0030036' because the actin cytoskeleton is defined as actin filaments and associated proteins. Relationships: is a type of actin cytoskeleton organization [GO:0030036] Subtypes: female germline ring canal stabilization [GO:0008335], myofibril assembly [GO:0030239], stress fiber assembly [GO:0043149], GO:0044837, sarcomere organization [GO:0045214], sarcomerogenesis [GO:0048769], GO:0106036 Regulation: RO_0002211 by GO:0110020